regulation of sporulation [GO:0043937] (biological process) Subtypes: GO:0034305, regulation of sexual sporulation [GO:0034306], GO:0042173, positive regulation of sporulation [GO:0043938], negative regulation of sporulation [GO:0043939] Sources: GOC:pamgo_curators Definition: Any process that modulates the frequency, rate or extent of sporulation, the process whose specific outcome is the progression of a spore over time, from its initiation to the mature structure. Relationships: is a type of regulation of developmental process [GO:0050793]; regulates sporulation [GO:0043934]